{
  "gene": "UniProtKB:P78363",
  "term_id": "GO:0140326",
  "term_label": "ATPase-coupled intramembrane lipid transporter activity",
  "gene_symbol": "ABCA4",
  "gene_name": "Retinal-specific phospholipid-transporting ATPase ABCA4"
}